{
  "term_label": "positive regulation of actin filament polymerization",
  "term_id": "GO:0030838",
  "gene": "UniProtKB:Q00587",
  "gene_name": "Cdc42 effector protein 1",
  "gene_symbol": "CDC42EP1"
}